4-hydroxybenzoate 4-O-beta-D-glucosyltransferase activity [GO:0047250] (molecular function) Definition: Catalysis of the reaction: 4-hydroxybenzoate + UDP-D-glucose = 4-(beta-D-glucosyloxy)benzoate + H+ + UDP. Sources: EC:2.4.1.194, RHEA:15153 Also known as: HBA glucosyltransferase activity, PHB glucosyltransferase activity, PHB-O-glucosyltransferase activity, UDP-glucose:4-(beta-D-glucopyranosyloxy)benzoic acid glucosyltransferase activity, UDP-glucose:4-hydroxybenzoate 4-O-beta-D-glucosyltransferase activity, UDPglucose:4-hydroxybenzoate 4-O-beta-D-glucosyltransferase activity, p-hydroxybenzoate glucosyltransferase activity, uridine diphosphoglucose-4-hydroxybenzoate glucosyltransferase activity Relationships: is a type of UDP-glucosyltransferase activity [GO:0035251]